{
  "term_id": "GO:0007264",
  "gene_name": "Rho guanine nucleotide exchange factor 18 (Fragment)",
  "term_label": "small GTPase-mediated signal transduction",
  "gene_symbol": "ARHGEF18",
  "gene": "UniProtKB:A0A590UK10"
}